{
  "gene_symbol": "FOXI3",
  "gene": "UniProtKB:A8MTJ6",
  "term_id": "GO:0030154",
  "gene_name": "Forkhead box protein I3",
  "term_label": "cell differentiation"
}